{
  "term_id": "GO:0016020",
  "gene": "UniProtKB:Q9UGF7",
  "gene_name": "Olfactory receptor 12D3",
  "gene_symbol": "OR12D3",
  "term_label": "membrane"
}